{
  "gene_name": "Krueppel-like factor 7",
  "gene": "UniProtKB:O75840",
  "term_label": "RNA polymerase II cis-regulatory region sequence-specific DNA binding",
  "term_id": "GO:0000978",
  "gene_symbol": "KLF7"
}